{
  "gene_name": "UDP-glucuronosyltransferase 1A1",
  "term_id": "GO:0008194",
  "gene_symbol": "UGT1A1",
  "term_label": "UDP-glycosyltransferase activity",
  "gene": "UniProtKB:P22309"
}